{
  "term_label": "Unknown biological process",
  "term_id": "UNKNOWN:0002",
  "gene_name": "Transmembrane protein 217",
  "gene": "UniProtKB:Q8N7C4",
  "gene_symbol": "TMEM217"
}